positive regulation of type I interferon production [GO:0032481] (biological process) Definition: Any process that activates or increases the frequency, rate, or extent of type I interferon production. Type I interferons include the interferon-alpha, beta, delta, episilon, zeta, kappa, tau, and omega gene families. Sources: GOC:add, GOC:mah Also known as: positive regulation of type I IFN production, up regulation of type I interferon production, up-regulation of type I interferon production, upregulation of type I interferon production, activation of type I interferon production, stimulation of type I interferon production Relationships: is a type of positive regulation of cytokine production [GO:0001819]; is a type of regulation of type I interferon production [GO:0032479]; positively regulates GO:0032606 Subtypes: positive regulation of interferon-alpha production [GO:0032727], GO:0032728